{
  "gene_symbol": "SLC25A27",
  "gene": "UniProtKB:O95847",
  "term_id": "GO:0009409",
  "term_label": "response to cold",
  "gene_name": "Mitochondrial uncoupling protein 4"
}